{
  "gene": "UniProtKB:Q8NI77",
  "term_label": "microtubule depolymerization",
  "gene_symbol": "KIF18A",
  "term_id": "GO:0007019",
  "gene_name": "Kinesin-like protein KIF18A"
}